{
  "gene": "UniProtKB:P02795",
  "term_label": "cellular response to cadmium ion",
  "gene_symbol": "MT2A",
  "gene_name": "Metallothionein-2",
  "term_id": "GO:0071276"
}